sex differentiation [GO:0007548] (biological process) Relationships: is a type of developmental process involved in reproduction [GO:0003006] Subtypes: GO:0046660, male sex differentiation [GO:0046661] Sources: GOC:ai Definition: The establishment of the sex of an organism by physical differentiation.